mitotic nuclear bridge midzone [GO:0140512] (cellular component) Definition: The central region of a mitotic nuclear bridge, distal to the main portions of the daughter nuclei. Relationships: is a type of cellular anatomical structure [GO:0110165]; is part of mitotic nuclear bridge [GO:0140510] References: PMID:32848252